{
  "term_id": "UNKNOWN:0002",
  "gene_symbol": "TDRD10",
  "gene_name": "Tudor domain-containing protein 10",
  "gene": "UniProtKB:Q5VZ19",
  "term_label": "Unknown biological process"
}